{
  "gene_symbol": "RAD51",
  "term_id": "GO:0042148",
  "term_label": "DNA strand invasion",
  "gene_name": "DNA repair protein RAD51 homolog 1",
  "gene": "UniProtKB:Q06609"
}